{
  "gene_symbol": "ZBTB14",
  "term_id": "GO:0000978",
  "term_label": "RNA polymerase II cis-regulatory region sequence-specific DNA binding",
  "gene_name": "Zinc finger and BTB domain-containing protein 14",
  "gene": "UniProtKB:O43829"
}